{
  "gene": "UniProtKB:Q9Y2M0",
  "term_id": "GO:0008409",
  "gene_name": "Fanconi-associated nuclease 1",
  "term_label": "5'-3' exonuclease activity",
  "gene_symbol": "FAN1"
}